positive regulation of cell projection organization [GO:0031346] (biological process) Sources: GOC:mah Subtypes: positive regulation of neuron projection development [GO:0010976], positive regulation of axonogenesis [GO:0050772], GO:0050775, positive regulation of plasma membrane bounded cell projection assembly [GO:0120034], GO:0150012, GO:1902210, positive regulation of lamellipodium organization [GO:1902745], GO:1902952, positive regulation of type IV pilus biogenesis [GO:1903658], positive regulation of microvillus length [GO:1903983] Also known as: positive regulation of cell projection organisation, up regulation of cell projection organization, up-regulation of cell projection organization, upregulation of cell projection organization, activation of cell projection organization, stimulation of cell projection organization, positive regulation of cell projection organization and biogenesis Relationships: is a type of GO:0031344; is a type of GO:0051130; positively regulates cell projection organization [GO:0030030] Definition: Any process that activates or increases the frequency, rate or extent of the process involved in the formation, arrangement of constituent parts, or disassembly of cell projections.